{
  "gene_name": "Protein HEXIM2",
  "gene": "UniProtKB:Q96MH2",
  "term_label": "cyclin-dependent protein serine/threonine kinase inhibitor activity",
  "term_id": "GO:0004861",
  "gene_symbol": "HEXIM2"
}